hydroxycyclohexanecarboxylate dehydrogenase activity [GO:0047010] (molecular function) Definition: Catalysis of the reaction: (1S,3R,4S)-3,4-dihydroxycyclohexane-1-carboxylate + NAD+ = (1S,4S)-4-hydroxy-3-oxocyclohexane-1-carboxylate + H+ + NADH. Sources: EC:1.1.1.166, RHEA:10516 Also known as: (-)t-3,t-4-dihydroxycyclohexane-c-1-carboxylate-NAD oxidoreductase activity, (1S,3R,4S)-3,4-dihydroxycyclohexane-1-carboxylate:NAD+ 3-oxidoreductase activity, dihydroxycyclohexanecarboxylate dehydrogenase activity Relationships: is a type of oxidoreductase activity, acting on the CH-OH group of donors, NAD or NADP as acceptor [GO:0016616]